{
  "gene_name": "Transmembrane protein CCDC163",
  "gene_symbol": "CCDC163",
  "term_label": "Unknown biological process",
  "term_id": "UNKNOWN:0002",
  "gene": "UniProtKB:A0A0D9SF12"
}